{
  "term_id": "GO:0003688",
  "term_label": "DNA replication origin binding",
  "gene_symbol": "ORC2",
  "gene_name": "Origin recognition complex subunit 2",
  "gene": "UniProtKB:Q13416"
}